{
  "term_id": "GO:0071816",
  "term_label": "tail-anchored membrane protein insertion into ER membrane",
  "gene": "UniProtKB:Q9Y3B6",
  "gene_symbol": "EMC9",
  "gene_name": "ER membrane protein complex subunit 9"
}